{
  "term_id": "GO:0043066",
  "term_label": "negative regulation of apoptotic process",
  "gene_symbol": "AKT2",
  "gene_name": "RAC-beta serine_threonine-protein kinase",
  "gene": "UniProtKB:P31751"
}